{
  "gene": "UniProtKB:Q9NVW2",
  "gene_symbol": "RLIM",
  "gene_name": "E3 ubiquitin-protein ligase RLIM",
  "term_id": "GO:0061630",
  "term_label": "ubiquitin protein ligase activity"
}